{
  "term_label": "Unknown molecular function",
  "term_id": "UNKNOWN:0001",
  "gene_name": "NADH dehydrogenase [ubiquinone] 1 beta subcomplex subunit 9",
  "gene_symbol": "NDUFB9",
  "gene": "UniProtKB:Q9Y6M9"
}